{
  "gene_symbol": "GABRR3",
  "term_id": "GO:1902476",
  "gene_name": "Gamma-aminobutyric acid receptor subunit rho-3",
  "term_label": "chloride transmembrane transport",
  "gene": "UniProtKB:A8MPY1"
}